nuclear polyadenylation-dependent rRNA catabolic process [GO:0071035] (biological process) Definition: The chemical reactions and pathways occurring in the nucleus and resulting in the breakdown of a ribosomal RNA (rRNA) molecule, including RNA fragments released as part of processing the primary transcript into multiple mature rRNA species, initiated by the enzymatic addition of a sequence of adenylyl residues (polyadenylation) at the 3' end the target rRNA. References: PMID:15173578, PMID:15572680, PMID:15935758, PMID:17652137, PMID:18591258 Sources: GOC:dgf, GOC:krc Also known as: nuclear poly(A)-dependent rRNA catabolic process Relationships: is a type of nuclear RNA surveillance [GO:0071027]